{
  "term_label": "Unknown molecular function",
  "gene_symbol": "UTP3",
  "term_id": "UNKNOWN:0001",
  "gene": "UniProtKB:Q9NQZ2",
  "gene_name": "Something about silencing protein 10"
}